{
  "gene": "UniProtKB:Q13315",
  "term_label": "negative regulation of TORC1 signaling",
  "term_id": "GO:1904262",
  "gene_name": "Serine-protein kinase ATM",
  "gene_symbol": "ATM"
}